{
  "term_id": "GO:0007186",
  "gene_name": "G-protein coupled receptor 35",
  "gene_symbol": "GPR35",
  "gene": "UniProtKB:Q9HC97",
  "term_label": "G protein-coupled receptor signaling pathway"
}